inositol-3-diphosphate-1,2,4,5,6-pentakisphosphate diphosphatase activity [GO:0052844] (molecular function) Definition: Catalysis of the reaction: 3-diphospho-1D-myo-inositol 1,2,4,5,6-pentakisphosphate + H2O = 1D-myo-inositol 1,2,3,4,5,6-hexakisphosphate + phosphate + 2 H+. References: PMID:10827188, PMID:11502751 Relationships: is a type of inositol diphosphate pentakisphosphate diphosphatase activity [GO:0052842]